{
  "gene_symbol": "NLRP11",
  "term_label": "cytoplasm",
  "term_id": "GO:0005737",
  "gene_name": "NACHT, LRR and PYD domains-containing protein 11",
  "gene": "UniProtKB:P59045"
}